{
  "gene": "UniProtKB:Q86XG9",
  "gene_symbol": "NBPF5P",
  "term_id": "UNKNOWN:0001",
  "gene_name": "Putative neuroblastoma breakpoint family member 5",
  "term_label": "Unknown molecular function"
}